{
  "term_id": "GO:0016607",
  "gene": "UniProtKB:Q96QD9",
  "gene_symbol": "FYTTD1",
  "gene_name": "UAP56-interacting factor",
  "term_label": "nuclear speck"
}